cholesterol 24-hydroxylase activity [GO:0033781] (molecular function) Definition: Catalysis of the reaction: cholesterol + H+ + NADPH + O2 = (24S)-24-hydroxycholesterol + H2O + NADP+. Sources: EC:1.14.14.25, RHEA:22716 Also known as: CYP46, CYP46A1, cholesterol 24-monooxygenase activity, cholesterol 24S-hydroxylase activity, cholesterol,NADPH:oxygen oxidoreductase (24-hydroxylating) activity, cytochrome P450 46A1 Relationships: is a type of oxidoreductase activity, acting on paired donors, with incorporation or reduction of molecular oxygen, NAD(P)H as one donor, and incorporation of one atom of oxygen [GO:0016709]